{
  "gene_symbol": "PLA2G4B",
  "gene": "UniProtKB:P0C869",
  "gene_name": "Cytosolic phospholipase A2 beta",
  "term_id": "GO:0047498",
  "term_label": "calcium-dependent phospholipase A2 activity"
}